{
  "term_label": "regulation of transcription by RNA polymerase II",
  "gene_symbol": "FOXJ2",
  "term_id": "GO:0006357",
  "gene_name": "Forkhead box protein J2",
  "gene": "UniProtKB:Q9P0K8"
}